positive regulation of extraocular skeletal muscle development [GO:0014727] (biological process) Relationships: is a type of regulation of extraocular skeletal muscle development [GO:0014725]; is a type of positive regulation of skeletal muscle tissue development [GO:0048643]; positively regulates extraocular skeletal muscle development [GO:0002074] Sources: GOC:mtg_muscle Definition: Any process that activates, maintains or increases the frequency, rate or extent of extraocular skeletal muscle development. Extraocular skeletal muscle development is the process whose specific outcome is the progression of the extraocular skeletal muscle over time, from its formation to the mature structure. The extraocular muscle is derived from cranial mesoderm and controls eye movements. The muscle begins its development with the differentiation of the muscle cells and ends with the mature muscle.